{
  "gene": "UniProtKB:P26368",
  "gene_symbol": "U2AF2",
  "term_label": "U2AF complex",
  "term_id": "GO:0089701",
  "gene_name": "Splicing factor U2AF 65 kDa subunit"
}